negative regulation of epidermal growth factor receptor signaling pathway [GO:0042059] (biological process) Also known as: down regulation of epidermal growth factor receptor signaling pathway, down-regulation of epidermal growth factor receptor signaling pathway, downregulation of epidermal growth factor receptor signaling pathway, negative regulation of EGF receptor signaling pathway, negative regulation of EGF receptor signalling pathway, negative regulation of EGFR signaling pathway, inhibition of epidermal growth factor receptor signaling pathway Relationships: is a type of GO:0042058; is a type of negative regulation of ERBB signaling pathway [GO:1901185]; RO_0002212 epidermal growth factor receptor signaling pathway [GO:0007173] Subtypes: epidermal growth factor catabolic process [GO:0007174], negative regulation of epidermal growth factor-activated receptor activity [GO:0007175], GO:1905283 Definition: Any process that stops, prevents, or reduces the frequency, rate or extent of epidermal growth factor receptor signaling pathway activity. Sources: GOC:go_curators